{
  "term_id": "UNKNOWN:0002",
  "gene_name": "Liver-expressed antimicrobial peptide 2",
  "gene": "UniProtKB:Q969E1",
  "gene_symbol": "LEAP2",
  "term_label": "Unknown biological process"
}